interleukin-33-mediated signaling pathway [GO:0038172] (biological process) Definition: The series of molecular signals initiated by interleukin-33 binding to its receptor on the surface of a target cell, and ending with the regulation of a downstream cellular process, e.g. transcription. Sources: GOC:jc, GOC:signaling Relationships: is a type of cytokine-mediated signaling pathway [GO:0019221] Also known as: IL-33-mediated signaling pathway, IL33 signaling pathway, interleukin-33-mediated signalling pathway, interleukin-33 signaling pathway